negative regulation of formation by symbiont of haustorium for nutrient acquisition from host [GO:0075047] (biological process) Definition: Any process that stops, prevents, or reduces the frequency, rate or extent of symbiont haustorium formation for nutrient acquisition from host. The host is defined as the larger of the organisms involved in a symbiotic interaction. Sources: GOC:pamgo_curators Note: Note that this term should not be used to annotate gene products of the host. It should only be used to annotate those gene products from the symbiont involved in this process. Relationships: is a type of GO:0044147; is a type of regulation of formation by symbiont of haustorium for nutrient acquisition from host [GO:0075045]; negatively regulates formation of haustorium for nutrient acquisition [GO:0052094]